{
  "term_id": "GO:0007200",
  "gene_name": "Lutropin-choriogonadotropic hormone receptor",
  "gene": "UniProtKB:P22888",
  "gene_symbol": "LHCGR",
  "term_label": "phospholipase C-activating G protein-coupled receptor signaling pathway"
}